negative regulation of monopolar cell growth [GO:0051514] (biological process) Definition: Any process that stops, prevents, or reduces the frequency, rate or extent of monopolar cell growth, polarized growth from one end of a cell. Sources: GOC:ai Also known as: down regulation of monopolar cell growth, down-regulation of monopolar cell growth, downregulation of monopolar cell growth, inhibition of monopolar cell growth Relationships: is a type of negative regulation of unidimensional cell growth [GO:0051511]; is a type of GO:0051513; negatively regulates GO:0042814 Subtypes: termination of monopolar cell growth [GO:0051521]